{
  "term_label": "plasma membrane",
  "gene_symbol": "CNTNAP3",
  "gene": "UniProtKB:Q9BZ76",
  "term_id": "GO:0005886",
  "gene_name": "Contactin-associated protein-like 3"
}